{
  "gene_symbol": "CACNA1E",
  "gene": "UniProtKB:Q15878",
  "gene_name": "Voltage-dependent R-type calcium channel subunit alpha-1E",
  "term_id": "GO:0008331",
  "term_label": "high voltage-gated calcium channel activity"
}